{
  "gene_symbol": "FCN1",
  "gene": "UniProtKB:O00602",
  "gene_name": "Ficolin-1",
  "term_id": "GO:0001867",
  "term_label": "complement activation, lectin pathway"
}